glycoprotein complex [GO:0090665] (CC) Definition: A protein complex containing at least one glycosylated protein, may be held together by both covalent and noncovalent bonds. Relationships: is a type of protein-containing complex [GO:0032991] Subtypes: dystrophin-associated glycoprotein complex [GO:0016010], alphaIIb-beta3 integrin-CD9-CD47-platelet glycoprotein Ib complex [GO:0071086], glycoprotein Ib-IX-V complex [GO:1990779] References: PMID:7693675, PMID:8662961 Sources: GOC:pf Note: An example is the Dictyostelium multi protein pspB complex, which is secreted from prespore vesicles and incorporated into the spore coat.